{
  "term_label": "plasma membrane",
  "gene_name": "Prolow-density lipoprotein receptor-related protein 1",
  "gene": "UniProtKB:Q07954",
  "gene_symbol": "LRP1",
  "term_id": "GO:0005886"
}